negative regulation of cell fate determination [GO:1905934] (biological process) Also known as: down regulation of cell fate determination, down-regulation of cell fate determination, downregulation of cell fate determination, inhibition of cell fate determination Definition: Any process that stops, prevents or reduces the frequency, rate or extent of cell fate determination. References: PMID:25793578 Sources: GOC:TermGenie, GOC:bhm, GO_REF:0000058 Subtypes: negative regulation of mesodermal cell fate determination [GO:0048335] Relationships: is a type of negative regulation of cell fate commitment [GO:0010454]; is a type of regulation of cell fate determination [GO:1905933]; negatively regulates cell fate determination [GO:0001709]